{
  "gene_symbol": "SKA2",
  "gene_name": "Spindle and kinetochore-associated protein 2",
  "term_id": "GO:0000278",
  "gene": "UniProtKB:Q8WVK7",
  "term_label": "mitotic cell cycle"
}